{
  "gene": "UniProtKB:Q9BWP8",
  "gene_symbol": "COLEC11",
  "term_id": "UNKNOWN:0002",
  "term_label": "Unknown biological process",
  "gene_name": "Collectin-11"
}